{
  "gene_name": "ADP-dependent glucokinase",
  "gene_symbol": "ADPGK",
  "gene": "UniProtKB:Q9BRR6",
  "term_label": "endoplasmic reticulum",
  "term_id": "GO:0005783"
}